{
  "term_label": "peroxisomal membrane",
  "term_id": "GO:0005778",
  "gene_name": "Mitochondrial fission 1 protein",
  "gene": "UniProtKB:Q9Y3D6",
  "gene_symbol": "FIS1"
}